{
  "term_label": "action potential",
  "gene": "UniProtKB:Q16322",
  "gene_symbol": "KCNA10",
  "gene_name": "Potassium voltage-gated channel subfamily A member 10",
  "term_id": "GO:0001508"
}